{
  "gene_name": "Refilin-A",
  "gene_symbol": "RFLNA",
  "term_id": "GO:0061182",
  "term_label": "negative regulation of chondrocyte development",
  "gene": "UniProtKB:Q6ZTI6"
}